{
  "term_id": "GO:0061630",
  "gene_symbol": "RNF31",
  "gene": "UniProtKB:Q96EP0",
  "term_label": "ubiquitin protein ligase activity",
  "gene_name": "E3 ubiquitin-protein ligase RNF31"
}